{
  "term_label": "Unknown biological process",
  "gene": "UniProtKB:Q9H7T3",
  "gene_symbol": "C10orf95",
  "gene_name": "Uncharacterized protein C10orf95",
  "term_id": "UNKNOWN:0002"
}